L-methionine biosynthetic process [GO:0071265] (biological process) Also known as: L-methionine anabolism, L-methionine biosynthesis, L-methionine formation, L-methionine synthesis Sources: GOC:ecd Definition: The chemical reactions and pathways resulting in the formation of L-methionine, the L-enantiomer of (2S)-2-amino-4-(methylsulfanyl)butanoic acid. Subtypes: L-methionine biosynthetic process from L-homoserine via O-acetyl-L-homoserine [GO:0019280], 'de novo' L-methionine biosynthetic process [GO:0071266], L-methionine salvage [GO:0071267] Relationships: is a type of methionine biosynthetic process [GO:0009086]